{
  "term_id": "GO:0005783",
  "gene_name": "Dolichol phosphate-mannose biosynthesis regulatory protein",
  "term_label": "endoplasmic reticulum",
  "gene": "UniProtKB:O94777",
  "gene_symbol": "DPM2"
}